{
  "gene_symbol": "ANGEL2",
  "gene_name": "Protein angel homolog 2",
  "term_label": "3'-UTR-mediated mRNA stabilization",
  "term_id": "GO:0070935",
  "gene": "UniProtKB:Q5VTE6"
}